{
  "gene_symbol": "JUNB",
  "gene": "UniProtKB:P17275",
  "term_id": "GO:0005667",
  "term_label": "transcription regulator complex",
  "gene_name": "Transcription factor JunB"
}